nitroquinoline-N-oxide reductase [NAD(P)H] activity [GO:0050465] (molecular function) Relationships: is a type of oxidoreductase activity, acting on other nitrogenous compounds as donors, with NAD or NADP as acceptor [GO:0046857] Definition: Catalysis of the reaction: 4-(hydroxyamino)quinoline N-oxide + 2 NAD(P)+ + H2O = 4-nitroquinoline N-oxide + 2 NAD(P)H + 2 H+. Sources: EC:1.7.1.9 Also known as: 4-(hydroxyamino)quinoline N-oxide:NADP+ oxidoreductase activity, 4-nitroquinoline 1-oxide reductase activity, 4NQO reductase activity, NAD(P)H2:4-nitroquinoline-N-oxide oxidoreductase activity, NAD(P)H:4-nitroquinoline-N-oxide oxidoreductase activity